{
  "term_label": "Unknown cellular component",
  "gene": "UniProtKB:Q5T749",
  "term_id": "UNKNOWN:0003",
  "gene_name": "Keratinocyte proline-rich protein",
  "gene_symbol": "KPRP"
}